{
  "gene_name": "Axonemal dynein light chain domain-containing protein 1",
  "gene_symbol": "AXDND1",
  "term_label": "Unknown molecular function",
  "gene": "UniProtKB:Q5T1B0",
  "term_id": "UNKNOWN:0001"
}